gas vesicle [GO:0031411] (cellular component) Also known as: gas vacuole References: PMID:22147705, PMID:8177173 Relationships: is_a intracellular membraneless organelle [GO:0043232] Note: Note that although this organelle is commonly referred to as a 'vesicle' or 'vacuole' in the literature, it is not surrounded by a membrane. Definition: An intracellular non-membrane-bounded organelle; a hollow structure made of protein, which usually has the form of a cylindrical tube closed by conical end caps. By regulating their relative gas vesicle content, aquatic microbes are able to perform vertical migrations.